{
  "gene_symbol": "KCT2",
  "gene": "UniProtKB:Q8NC54",
  "gene_name": "Keratinocyte-associated transmembrane protein 2",
  "term_label": "Unknown molecular function",
  "term_id": "UNKNOWN:0001"
}